negative regulation of neuroblast proliferation [GO:0007406] (biological process) Definition: Any process that stops, prevents, or reduces the frequency, rate or extent of the proliferation of neuroblasts. Sources: GOC:ai Relationships: is a type of negative regulation of neurogenesis [GO:0050768]; is a type of regulation of neuroblast proliferation [GO:1902692]; is a type of negative regulation of neural precursor cell proliferation [GO:2000178]; negatively regulates GO:0007405 Also known as: down regulation of neuroblast proliferation, down-regulation of neuroblast proliferation, downregulation of neuroblast proliferation, suppression of neuroblast proliferation, inhibition of neuroblast proliferation